positive regulation of T cell mediated immune response to tumor cell [GO:0002842] (biological process) Sources: GOC:add Relationships: is a type of positive regulation of T cell mediated immunity [GO:0002711]; is a type of positive regulation of immune response to tumor cell [GO:0002839]; is_a regulation of T cell mediated immune response to tumor cell [GO:0002840]; positively regulates T cell mediated immune response to tumor cell [GO:0002424] Also known as: positive regulation of T cell mediated immune response to tumour cell, positive regulation of T lymphocyte mediated immune response to tumor cell, positive regulation of T-cell mediated immune response to tumor cell, positive regulation of T-lymphocyte mediated immune response to tumor cell, up regulation of T cell mediated immune response to tumor cell, up-regulation of T cell mediated immune response to tumor cell, upregulation of T cell mediated immune response to tumor cell, activation of T cell mediated immune response to tumor cell, stimulation of T cell mediated immune response to tumor cell Subtypes: positive regulation of T cell tolerance induction to tumor cell [GO:0002848], positive regulation of T cell mediated cytotoxicity directed against tumor cell target [GO:0002854] Definition: Any process that activates or increases the frequency, rate, or extent of a T cell mediated immune response to tumor cell.